{
  "term_id": "GO:0050808",
  "gene_name": "Hemicentin-2",
  "gene_symbol": "HMCN2",
  "term_label": "synapse organization",
  "gene": "UniProtKB:Q8NDA2"
}